positive regulation of skeletal muscle hypertrophy [GO:1904206] (biological process) Relationships: is_a positive regulation of muscle hypertrophy [GO:0014742]; is a type of positive regulation of muscle adaptation [GO:0014744]; is a type of regulation of skeletal muscle hypertrophy [GO:1904204]; positively regulates skeletal muscle hypertrophy [GO:0014734] References: PMID:23470307 Sources: GOC:TermGenie, GO_REF:0000058 Also known as: up regulation of skeletal muscle hypertrophy, up-regulation of skeletal muscle hypertrophy, upregulation of skeletal muscle hypertrophy, activation of skeletal muscle hypertrophy Definition: Any process that activates or increases the frequency, rate or extent of skeletal muscle hypertrophy.